{
  "gene": "UniProtKB:Q7RTV3",
  "term_label": "regulation of transcription by RNA polymerase II",
  "term_id": "GO:0006357",
  "gene_name": "Zinc finger protein 367",
  "gene_symbol": "ZNF367"
}